{
  "term_id": "GO:0033627",
  "gene": "UniProtKB:O95965",
  "gene_symbol": "ITGBL1",
  "gene_name": "Integrin beta-like protein 1",
  "term_label": "cell adhesion mediated by integrin"
}